{
  "gene_symbol": "GSTA5",
  "gene_name": "Glutathione S-transferase A5",
  "term_label": "cytosol",
  "term_id": "GO:0005829",
  "gene": "UniProtKB:Q7RTV2"
}